{
  "term_label": "Unknown cellular component",
  "gene_symbol": "IFI44L",
  "gene_name": "Interferon-induced protein 44-like",
  "gene": "UniProtKB:Q53G44",
  "term_id": "UNKNOWN:0003"
}